{
  "gene": "UniProtKB:P14138",
  "term_id": "GO:0005179",
  "gene_symbol": "EDN3",
  "gene_name": "Endothelin-3",
  "term_label": "hormone activity"
}